{
  "term_label": "Unknown molecular function",
  "gene": "UniProtKB:E0CX11",
  "gene_name": "Short transmembrane mitochondrial protein 1",
  "term_id": "UNKNOWN:0001",
  "gene_symbol": "STMP1"
}